high-affinity ferrous iron transmembrane transporter activity [GO:0061840] (molecular function) Definition: Enables the transfer of ferrous iron (Fe(II) or Fe2+) ions from one side of a membrane to the other. In high-affinity transport the transporter is able to bind the solute even if it is only present at very low concentrations. References: PMID:9413439 Sources: GOC:bhm Relationships: is a type of ferrous iron transmembrane transporter activity [GO:0015093] Also known as: high affinity ferrous uptake transmembrane transporter activity, high-affinity ferrous iron uptake transmembrane transporter activity